UDP metabolic process [GO:0046048] (biological process) Sources: GOC:go_curators Relationships: is a type of pyrimidine ribonucleoside diphosphate metabolic process [GO:0009193]; is a type of pyrimidine ribonucleotide metabolic process [GO:0009218] Also known as: UDP metabolism Definition: The chemical reactions and pathways involving UDP, uridine (5'-)diphosphate. Subtypes: UDP biosynthetic process [GO:0006225], UDP catabolic process [GO:0006256]